{
  "gene": "UniProtKB:P15121",
  "term_label": "cytosol",
  "term_id": "GO:0005829",
  "gene_symbol": "AKR1B1",
  "gene_name": "Aldo-keto reductase family 1 member B1"
}